mating type determination [GO:0007531] (biological process) Relationships: is_a sex determination [GO:0007530] Definition: Any process that establishes and transmits the specification of mating type upon an individual. Mating types are the equivalent in microorganisms of the sexes in higher organisms. References: PMID:28916791, PMID:33313646, PMID:8274857, PMID:8785123 Subtypes: regulation of mating-type specific transcription, DNA-templated [GO:0007532], GO:0007533